{
  "gene": "UniProtKB:O60925",
  "term_id": "GO:0005737",
  "term_label": "cytoplasm",
  "gene_name": "Prefoldin subunit 1",
  "gene_symbol": "PFDN1"
}